{
  "term_id": "GO:0005634",
  "gene_symbol": "GCHFR",
  "gene_name": "GTP cyclohydrolase 1 feedback regulatory protein",
  "term_label": "nucleus",
  "gene": "UniProtKB:P30047"
}